{
  "gene": "UniProtKB:A0A075B6J9",
  "term_label": "immunoglobulin complex",
  "gene_symbol": "IGLV2-18",
  "gene_name": "Immunoglobulin lambda variable 2-18",
  "term_id": "GO:0019814"
}